{
  "term_label": "RNA polymerase II cis-regulatory region sequence-specific DNA binding",
  "term_id": "GO:0000978",
  "gene_name": "Homeobox protein OTX1",
  "gene": "UniProtKB:P32242",
  "gene_symbol": "OTX1"
}